spindle assembly involved in male meiosis [GO:0007053] (biological process) Sources: GOC:mah Subtypes: spindle assembly involved in male meiosis I [GO:0007054], GO:0007055, anastral spindle assembly involved in male meiosis [GO:0009971] Relationships: is_a meiotic spindle assembly [GO:0090306]; is part of male meiotic nuclear division [GO:0007140] Definition: The aggregation, arrangement and bonding together of a set of components to form the spindle during a meiotic cell cycle in males. An example of this is found in Drosophila melanogaster.